{
  "term_label": "intracellular signal transduction",
  "gene_name": "Leucine-rich repeat protein SHOC-2",
  "gene": "UniProtKB:Q9UQ13",
  "gene_symbol": "SHOC2",
  "term_id": "GO:0035556"
}